negative regulation of RNA splicing [GO:0033119] (biological process) Relationships: is a type of GO:0010629; is a type of GO:0043484; RO_0002212 RNA splicing [GO:0008380] Definition: Any process that stops, prevents, or reduces the frequency, rate or extent of RNA splicing. Subtypes: negative regulation of mRNA splicing, via spliceosome [GO:0048025] Sources: GOC:mah